{
  "gene_symbol": "NCALD",
  "gene": "UniProtKB:P61601",
  "gene_name": "Neurocalcin-delta",
  "term_id": "GO:0009966",
  "term_label": "regulation of signal transduction"
}